{
  "gene_symbol": "DDIT4L",
  "gene_name": "DNA damage-inducible transcript 4-like protein",
  "term_id": "UNKNOWN:0001",
  "gene": "UniProtKB:Q96D03",
  "term_label": "Unknown molecular function"
}